{
  "gene_name": "Zinc finger protein 57",
  "term_label": "nucleus",
  "gene": "UniProtKB:Q68EA5",
  "gene_symbol": "ZNF57",
  "term_id": "GO:0005634"
}